ABC-type protein transporter activity [GO:0015462] (molecular function) Definition: Enables the transfer of a solute or solutes from one side of a membrane to the other according to the reaction: ATP + H2O + protein(out) = ADP + phosphate + protein(in). Sources: GOC:jl Note: Enzymes with this activity include bacterial enzymes dedicated to the secretion of one or several closely related proteins belonging to the toxin, protease and lipase families, for example alpha-hemolysin, cyclolysin, colicin V, siderophores, bacteriocin, subtilin, competence factor and pediocin (from EC:7.4.2.5). Also known as: protein-transporting ATPase activity, ABC-type protein transmembrane transporter activity, protein ABC transporter, pilin/fimbrilin exporter activity, ATPase-coupled protein transmembrane transporter activity, protein-transmembrane transporting ATPase activity Relationships: is a type of protein-transporting ATPase activity [GO:0015450]; is a type of GO:0140359